{
  "gene": "UniProtKB:Q06830",
  "gene_name": "Peroxiredoxin-1",
  "term_label": "cell redox homeostasis",
  "term_id": "GO:0045454",
  "gene_symbol": "PRDX1"
}